endocytic iron import into cell [GO:0140298] (biological process) Relationships: is a type of GO:0006898; is_a iron import into cell [GO:0033212] Definition: Uptake of iron into a cell via binding to an extracellular receptor, which is internalized by endocytosis. References: PMID:23092063 Also known as: iron import into cell by endocytosis Subtypes: endocytic heme import into cell [GO:0140421]